{
  "gene_symbol": "BEND6",
  "gene_name": "BEN domain-containing protein 6",
  "gene": "UniProtKB:Q5SZJ8",
  "term_label": "transcription corepressor activity",
  "term_id": "GO:0003714"
}